{
  "gene_symbol": "HROB",
  "term_label": "Unknown cellular component",
  "term_id": "UNKNOWN:0003",
  "gene": "UniProtKB:Q8N3J3",
  "gene_name": "Homologous recombination OB-fold protein"
}